{
  "gene_name": "SH2 domain-containing protein 5",
  "gene": "UniProtKB:Q6ZV89",
  "gene_symbol": "SH2D5",
  "term_id": "UNKNOWN:0002",
  "term_label": "Unknown biological process"
}